{
  "term_label": "alveolar lamellar body",
  "gene_symbol": "SFTPB",
  "gene_name": "Pulmonary surfactant-associated protein B",
  "term_id": "GO:0097208",
  "gene": "UniProtKB:P07988"
}